{
  "gene_symbol": "TAS2R20",
  "term_label": "membrane",
  "gene": "UniProtKB:P59543",
  "gene_name": "Taste receptor type 2 member 20",
  "term_id": "GO:0016020"
}